{
  "gene_name": "Semaphorin-3G",
  "term_label": "semaphorin-plexin signaling pathway",
  "gene": "UniProtKB:Q9NS98",
  "gene_symbol": "SEMA3G",
  "term_id": "GO:0071526"
}